{
  "gene_name": "Tumor necrosis factor ligand superfamily member 15",
  "gene_symbol": "TNFSF15",
  "term_label": "positive regulation of extrinsic apoptotic signaling pathway",
  "gene": "UniProtKB:O95150",
  "term_id": "GO:2001238"
}